{
  "term_label": "negative regulation of DNA-templated transcription",
  "gene": "UniProtKB:Q9UN30",
  "gene_name": "Sex comb on midleg-like protein 1",
  "gene_symbol": "SCML1",
  "term_id": "GO:0045892"
}